actin filament of cell cortex of cell tip [GO:1903145] (cellular component) References: PMID:20807799, PMID:24954052 Sources: GOC:TermGenie, GO_REF:0000064 Definition: Any actin filament that is part of a cell cortex of cell tip. Relationships: is a type of actin filament [GO:0005884]; is part of cell cortex of cell tip [GO:0051285] Also known as: actin filament of cell cortex of cell end, microfilament of cell cortex of cell end, microfilament of cell cortex of cell tip